procollagen-proline 4-dioxygenase complex, alpha(I) type [GO:0070386] (cellular component) Definition: A procollagen-proline 4-dioxygenase complex that contains alpha subunits of the type I isoform; its activity is readily inhibited by poly(L-proline). Also known as: prolyl 4-hydroxylase complex (alpha(I)-type), procollagen-proline, 2-oxoglutarate-4-dioxygenase complex, alpha(I) type References: PMID:14500733, PMID:7753822 Relationships: is_a procollagen-proline 4-dioxygenase complex [GO:0016222]